{
  "term_label": "signal transduction",
  "gene_symbol": "OR1L3",
  "term_id": "GO:0007165",
  "gene": "UniProtKB:Q8NH93",
  "gene_name": "Olfactory receptor 1L3"
}